negative regulation of artery morphogenesis [GO:1905652] (biological process) References: PMID:27389411 Sources: GOC:BHF, GOC:BHF_miRNA, GOC:TermGenie, GOC:rph, GO_REF:0000058 Relationships: is a type of regulation of artery morphogenesis [GO:1905651]; is a type of negative regulation of blood vessel morphogenesis [GO:2000181]; negatively regulates artery morphogenesis [GO:0048844] Definition: Any process that stops, prevents or reduces the frequency, rate or extent of artery morphogenesis. Also known as: down regulation of arterial morphogenesis, down regulation of arteriogenesis, down regulation of artery morphogenesis, down-regulation of arterial morphogenesis, down-regulation of arteriogenesis, down-regulation of artery morphogenesis, downregulation of arterial morphogenesis, downregulation of arteriogenesis, downregulation of artery morphogenesis, negative regulation of arterial morphogenesis, negative regulation of arteriogenesis, inhibition of arterial morphogenesis, inhibition of arteriogenesis, inhibition of artery morphogenesis Subtypes: negative regulation of aorta morphogenesis [GO:1903848], negative regulation of ductus arteriosus closure [GO:1904336]